{
  "term_label": "translation",
  "gene_name": "Small ribosomal subunit protein eS4, Y isoform 2",
  "term_id": "GO:0006412",
  "gene": "UniProtKB:Q8TD47",
  "gene_symbol": "RPS4Y2"
}